carpel structural organization [GO:0048463] (biological process) Sources: GOC:jid Also known as: carpel structural organisation Definition: The process that contributes to the act of creating the structural organization of the carpel. This process pertains to the physical shaping of a rudimentary structure. Relationships: is a type of GO:0048450; BFO_0000050 carpel morphogenesis [GO:0048445]